{
  "gene_name": "Uncharacterized protein C19orf85",
  "term_id": "UNKNOWN:0001",
  "gene": "UniProtKB:A0A1B0GUS0",
  "term_label": "Unknown molecular function",
  "gene_symbol": "C19orf85"
}